dCMP biosynthetic process [GO:0046064] (biological process) Relationships: is a type of pyrimidine deoxyribonucleoside monophosphate biosynthetic process [GO:0009177]; is a type of pyrimidine deoxyribonucleotide biosynthetic process [GO:0009221]; is a type of dCMP metabolic process [GO:0046063] Sources: GOC:go_curators Definition: The chemical reactions and pathways resulting in the formation of dCMP, deoxycytidine monophosphate. Also known as: dCMP anabolism, dCMP biosynthesis, dCMP formation, dCMP synthesis Subtypes: GO:0006239